{
  "term_label": "transcription coregulator activity",
  "gene_name": "AF4_FMR2 family member 2",
  "gene_symbol": "AFF2",
  "term_id": "GO:0003712",
  "gene": "UniProtKB:P51816"
}